negative regulation of lipid biosynthetic process [GO:0051055] (biological process) Definition: Any process that stops, prevents, or reduces the frequency, rate or extent of the chemical reactions and pathways resulting in the formation of lipids. Also known as: down regulation of lipid biosynthetic process, down-regulation of lipid biosynthetic process, downregulation of lipid biosynthetic process, negative regulation of lipid anabolism, negative regulation of lipid biosynthesis, negative regulation of lipid formation, negative regulation of lipid synthesis, negative regulation of lipogenesis, inhibition of lipid biosynthetic process Subtypes: negative regulation of gibberellin biosynthetic process [GO:0010373], negative regulation of triglyceride biosynthetic process [GO:0010868], negative regulation of steroid biosynthetic process [GO:0010894], negative regulation of fatty acid biosynthetic process [GO:0045717], negative regulation of juvenile hormone biosynthetic process [GO:0045968], GO:0071072, negative regulation of sphingolipid biosynthetic process [GO:0090155], negative regulation of abscisic acid biosynthetic process [GO:0090359], negative regulation of retinoic acid biosynthetic process [GO:1900053], negative regulation of diacylglycerol biosynthetic process [GO:1900481], negative regulation of butyryl-CoA catabolic process to butanol [GO:1900498], negative regulation of emericellamide biosynthetic process [GO:1900659], GO:1900948, negative regulation of ent-pimara-8(14),15-diene biosynthetic process [GO:1901543], negative regulation of carotenoid biosynthetic process [GO:1904142], negative regulation of wax biosynthetic process [GO:1904277] Sources: GOC:ai Relationships: is a type of GO:0009890; is a type of negative regulation of lipid metabolic process [GO:0045833]; is a type of regulation of lipid biosynthetic process [GO:0046890]; RO_0002212 lipid biosynthetic process [GO:0008610]